{
  "term_id": "GO:0015020",
  "gene_name": "UDP-glucuronosyltransferase 2B17",
  "term_label": "glucuronosyltransferase activity",
  "gene": "UniProtKB:O75795",
  "gene_symbol": "UGT2B17"
}